{
  "gene": "UniProtKB:O60732",
  "term_id": "GO:0005634",
  "gene_symbol": "MAGEC1",
  "term_label": "nucleus",
  "gene_name": "Melanoma-associated antigen C1"
}